{
  "gene_symbol": "ELP3",
  "gene_name": "Elongator complex protein 3",
  "term_label": "nucleus",
  "gene": "UniProtKB:Q9H9T3",
  "term_id": "GO:0005634"
}